{
  "gene_symbol": "SLA",
  "term_label": "nucleoplasm",
  "gene_name": "Src-like-adapter",
  "gene": "UniProtKB:Q13239",
  "term_id": "GO:0005654"
}